{
  "term_label": "Unknown cellular component",
  "gene": "UniProtKB:Q96RM1",
  "gene_symbol": "SPRR2F",
  "term_id": "UNKNOWN:0003",
  "gene_name": "Small proline-rich protein 2F"
}